{
  "gene_name": "Zinc finger protein 547",
  "gene": "UniProtKB:Q8IVP9",
  "term_id": "GO:0000981",
  "gene_symbol": "ZNF547",
  "term_label": "DNA-binding transcription factor activity, RNA polymerase II-specific"
}